{
  "gene_name": "Protein maelstrom homolog",
  "term_id": "GO:0034587",
  "gene": "UniProtKB:Q96JY0",
  "gene_symbol": "MAEL",
  "term_label": "piRNA processing"
}